{
  "term_label": "Unknown biological process",
  "term_id": "UNKNOWN:0002",
  "gene_name": "Interleukin-31",
  "gene_symbol": "IL31",
  "gene": "UniProtKB:Q6EBC2"
}